{
  "term_id": "UNKNOWN:0002",
  "gene_symbol": "ID2B",
  "gene": "UniProtKB:Q14602",
  "gene_name": "Putative DNA-binding protein inhibitor ID-2B",
  "term_label": "Unknown biological process"
}